{
  "gene_symbol": "ILK",
  "term_label": "substrate adhesion-dependent cell spreading",
  "term_id": "GO:0034446",
  "gene_name": "Integrin-linked protein kinase",
  "gene": "UniProtKB:Q13418"
}